{
  "gene": "UniProtKB:P03979",
  "term_id": "UNKNOWN:0002",
  "term_label": "Unknown biological process",
  "gene_name": "T cell receptor gamma variable 3",
  "gene_symbol": "TRGV3"
}